{
  "gene_symbol": "PDCD1LG2",
  "term_id": "GO:0006955",
  "term_label": "immune response",
  "gene": "UniProtKB:Q9BQ51",
  "gene_name": "Programmed cell death 1 ligand 2"
}